isopentenyl diphosphate biosynthetic process, mevalonate pathway involved in terpenoid biosynthetic process [GO:0051486] (biological process) Also known as: isopentenyl diphosphate anabolism, mevalonate pathway, during terpenoid anabolism, isopentenyl diphosphate biosynthetic process, mevalonate pathway, during terpenoid biosynthetic process, isopentenyl diphosphate formation, mevalonate pathway, during terpenoid biosynthesis, isopentenyl diphosphate formation, mevalonate pathway, during terpenoid formation, isopentenyl diphosphate synthesis, mevalonate pathway, during terpenoid synthesis Relationships: is a type of isopentenyl diphosphate biosynthetic process, mevalonate pathway [GO:0019287]; is part of terpenoid biosynthetic process, mevalonate-dependent [GO:0051485] Definition: The chemical reactions and pathways resulting in the formation of isopentenyl diphosphate by the mevalonate pathway that contributes to terpenoid biosynthesis. This pathway converts acetate, in the form of acetyl-CoA, to isopentenyl diphosphate (IPP) through a series of mevalonate intermediates. Sources: GOC:ai